{
  "gene_name": "Sentrin-specific protease 6",
  "gene": "UniProtKB:Q9GZR1",
  "term_id": "GO:0005634",
  "gene_symbol": "SENP6",
  "term_label": "nucleus"
}